{
  "gene_name": "Exocyst complex component 3",
  "gene": "UniProtKB:O60645",
  "gene_symbol": "EXOC3",
  "term_label": "exocyst",
  "term_id": "GO:0000145"
}